G protein-coupled chemoattractant receptor activity [GO:0001637] (MF) Relationships: is a type of G protein-coupled receptor activity [GO:0004930] Definition: Combining with a chemoattractant and transmitting the signal across the membrane by activating an associated G-protein; promotes the exchange of GDP for GTP on the alpha subunit of a heterotrimeric G-protein complex. Also known as: G protein chemoattractant receptor activity, G-protein chemoattractant receptor activity, G-protein coupled chemoattractant receptor activity Subtypes: chemokine receptor activity [GO:0004950] Sources: GOC:bf, GOC:mah